{
  "term_label": "cytokine activity",
  "gene_symbol": "GDF11",
  "term_id": "GO:0005125",
  "gene_name": "Growth_differentiation factor 11",
  "gene": "UniProtKB:O95390"
}